{
  "term_label": "chromatin binding",
  "gene_name": "ATPase family AAA domain-containing protein 2",
  "gene_symbol": "ATAD2",
  "term_id": "GO:0003682",
  "gene": "UniProtKB:Q6PL18"
}